regulation of membrane tubulation [GO:1903525] (biological process) Subtypes: GO:1903526, positive regulation of membrane tubulation [GO:1903527] Relationships: is a type of regulation of plasma membrane organization [GO:1903729]; regulates plasma membrane tubulation [GO:0097320] Definition: Any process that modulates the frequency, rate or extent of membrane tubulation. Also known as: regulation of plasma membrane tubulation, regulation of vesicle scission References: PMID:18388313 Sources: GOC:TermGenie, GOC:pm, GO_REF:0000058